{
  "gene_name": "Acyl-protein thioesterase 1",
  "gene_symbol": "LYPLA1",
  "gene": "UniProtKB:O75608",
  "term_label": "negative regulation of Golgi to plasma membrane protein transport",
  "term_id": "GO:0042997"
}